{
  "gene_symbol": "C1QC",
  "term_id": "UNKNOWN:0003",
  "gene": "UniProtKB:P02747",
  "gene_name": "Complement C1q subcomponent subunit C",
  "term_label": "Unknown cellular component"
}